{
  "gene_symbol": "RAD17",
  "term_id": "GO:0035861",
  "term_label": "site of double-strand break",
  "gene": "UniProtKB:O75943",
  "gene_name": "Cell cycle checkpoint protein RAD17"
}